mammillotectal axonal tract development [GO:0061375] (biological process) Definition: The progression of the mammillotectal tract over time, from its formation to the mature structure. The mammillotectal tract is the collection of axons that connects the ventral diencephalon to the superior colliculus. Relationships: is a type of anatomical structure development [GO:0048856]; is part of mammillary axonal complex development [GO:0061373] References: PMID:10662642 Sources: GOC:dph, GOC:yaf